{
  "gene": "UniProtKB:P25398",
  "gene_symbol": "RPS12",
  "term_id": "GO:1990145",
  "gene_name": "Small ribosomal subunit protein eS12",
  "term_label": "maintenance of translational fidelity"
}